fusion of sperm to egg plasma membrane involved in double fertilization forming a zygote and endosperm [GO:0061936] (biological process) Relationships: is a type of GO:0022412; is a type of plasma membrane fusion [GO:0045026]; is part of double fertilization forming a zygote and endosperm [GO:0009567] References: PMID:21123745 Definition: The binding and fusion of a sperm, with the plasma membrane of the oocyte as part of the process of double fertilization forming a zygote and endosperm.